{
  "term_label": "extracellular space",
  "term_id": "GO:0005615",
  "gene": "UniProtKB:P22692",
  "gene_symbol": "IGFBP4",
  "gene_name": "Insulin-like growth factor-binding protein 4"
}